{
  "term_id": "GO:0005886",
  "gene": "UniProtKB:P19440",
  "term_label": "plasma membrane",
  "gene_symbol": "GGT1",
  "gene_name": "Glutathione hydrolase 1 proenzyme"
}